{
  "term_label": "Unknown cellular component",
  "gene_symbol": "PTPRK",
  "gene": "UniProtKB:Q15262",
  "gene_name": "Receptor-type tyrosine-protein phosphatase kappa",
  "term_id": "UNKNOWN:0003"
}